{
  "gene_name": "Kynurenine formamidase",
  "gene": "UniProtKB:Q63HM1",
  "term_id": "GO:0019441",
  "gene_symbol": "AFMID",
  "term_label": "L-tryptophan catabolic process to kynurenine"
}